{
  "term_label": "membrane",
  "gene": "UniProtKB:P11021",
  "term_id": "GO:0016020",
  "gene_name": "Endoplasmic reticulum chaperone BiP",
  "gene_symbol": "HSPA5"
}